negative regulation of cardiac vascular smooth muscle cell differentiation [GO:2000723] (biological process) Relationships: is a type of negative regulation of vascular associated smooth muscle cell differentiation [GO:1905064]; is a type of negative regulation of cardiocyte differentiation [GO:1905208]; is a type of regulation of cardiac vascular smooth muscle cell differentiation [GO:2000722]; negatively regulates cardiac vascular smooth muscle cell differentiation [GO:0060947] Definition: Any process that stops, prevents or reduces the frequency, rate or extent of cardiac vascular smooth muscle cell differentiation. Also known as: negative regulation of heart vascular smooth muscle cell differentiation Sources: GOC:BHF